specification of metanephric connecting tubule identity [GO:0072294] (biological process) Definition: The process in which the connecting tubule of the metanephric nephron acquires its identity. Sources: GOC:bf, GOC:mtg_kidney_jan10 Relationships: is_a GO:0072085; is a type of specification of metanephric nephron tubule identity [GO:0072293]; is part of metanephric connecting tubule development [GO:0072286]